glutamate-tRNA ligase complex [GO:0009332] (cellular component) References: PMID:29679766 Definition: An enzyme complex that catalyzes the ligation of glutamate and tRNA(Glu) to form glutamyl-tRNA(Glu). Relationships: is a type of catalytic complex [GO:1902494]; is part of cytoplasm [GO:0005737]